{
  "term_id": "GO:0007283",
  "term_label": "spermatogenesis",
  "gene_symbol": "MAEL",
  "gene_name": "Protein maelstrom homolog",
  "gene": "UniProtKB:Q96JY0"
}